positive regulation of endothelial cell chemotaxis to vascular endothelial growth factor [GO:1904859] (biological process) References: PMID:21885851 Sources: GOC:BHF, GOC:BHF_miRNA, GOC:TermGenie, GOC:rph, GO_REF:0000058 Relationships: is a type of GO:0030335; is a type of positive regulation of chemotaxis [GO:0050921]; is a type of regulation of endothelial cell chemotaxis to vascular endothelial growth factor [GO:1904857]; positively regulates endothelial cell chemotaxis to vascular endothelial growth factor [GO:0090668] Definition: Any process that activates or increases the frequency, rate or extent of endothelial cell chemotaxis to vascular endothelial growth factor. Also known as: up regulation of endothelial cell chemotaxis to vascular endothelial growth factor, up-regulation of endothelial cell chemotaxis to vascular endothelial growth factor, upregulation of endothelial cell chemotaxis to vascular endothelial growth factor, activation of endothelial cell chemotaxis to vascular endothelial growth factor